adenylate cyclase-activating serotonin receptor signaling pathway [GO:0007192] (biological process) Also known as: serotonin receptor, adenylyl cyclase activating pathway, activation of adenylate cyclase activity by serotonin receptor signalling pathway, serotonin receptor, adenylate cyclase activating pathway Sources: GOC:dph, GOC:mah, GOC:signaling, GOC:tb Definition: An adenylate cyclase-activating G protein-coupled receptor signaling pathway initiated by serotonin binding to its receptor, and ending with the regulation of a downstream cellular process. Relationships: is a type of GO:0007189; is a type of serotonin receptor signaling pathway [GO:0007210]